{
  "term_id": "GO:0005654",
  "gene_name": "Zinc finger and BTB domain-containing protein 2",
  "term_label": "nucleoplasm",
  "gene_symbol": "ZBTB2",
  "gene": "UniProtKB:Q8N680"
}